integrin alphaD-beta2 complex [GO:0034690] (cellular component) References: PMID:12297042 Also known as: alphaD-beta2 integrin complex, Itgad-Itgb2 complex Definition: An integrin complex that comprises one alphaD subunit and one beta2 subunit. Relationships: is a type of integrin complex [GO:0008305]